cytosolic electron transfer flavoprotein complex [GO:0045247] (cellular component) Relationships: is a type of electron transfer flavoprotein complex [GO:0045251]; BFO_0000050 cytosol [GO:0005829] Definition: A protein complex located in the cytosol containing flavin adenine dinucleotide (FAD) that, together with an acyl-CoA dehydrogenase, forms a system that oxidizes an acyl-CoA molecule and reduces ubiquinone and other acceptors. Sources: GOC:mtg_sensu, ISBN:0198506732